neuroblast division in pallium [GO:0022017] (biological process) Definition: The division of neuroblasts in the pallium. Neuroblasts are precursor cells that give rise to neurons. Sources: GOC:cls, GOC:dgh, GOC:dph, GOC:jid, GO_REF:0000021 Relationships: is a type of forebrain neuroblast division [GO:0021873]; is part of pallium cell proliferation in forebrain [GO:0022013]